{
  "gene_symbol": "PFKP",
  "term_id": "GO:0003872",
  "gene": "UniProtKB:Q01813",
  "gene_name": "ATP-dependent 6-phosphofructokinase, platelet type",
  "term_label": "6-phosphofructokinase activity"
}